{
  "gene": "UniProtKB:Q9NZT2",
  "term_id": "UNKNOWN:0001",
  "gene_symbol": "OGFR",
  "gene_name": "Opioid growth factor receptor",
  "term_label": "Unknown molecular function"
}